cytosolic large ribosomal subunit assembly [GO:0180023] (biological process) Definition: The aggregation, arrangement and bonding together of a set of components to form a cytosolic large ribosomal subunit. Relationships: is a type of GO:0000027; is part of GO:0042256 References: PMID:30467428